{
  "gene_name": "Arachidonate 5-lipoxygenase-activating protein",
  "gene_symbol": "ALOX5AP",
  "gene": "UniProtKB:P20292",
  "term_label": "glutathione transferase activity",
  "term_id": "GO:0004364"
}